{
  "gene": "UniProtKB:Q16181",
  "term_id": "GO:0008104",
  "gene_symbol": "SEPTIN7",
  "gene_name": "Septin-7",
  "term_label": "intracellular protein localization"
}